{
  "term_id": "GO:0046854",
  "gene": "UniProtKB:Q9UHH9",
  "gene_symbol": "IP6K2",
  "gene_name": "Inositol hexakisphosphate kinase 2",
  "term_label": "phosphatidylinositol phosphate biosynthetic process"
}